{
  "term_label": "sulfation",
  "gene": "UniProtKB:P49888",
  "gene_name": "Sulfotransferase 1E1",
  "gene_symbol": "SULT1E1",
  "term_id": "GO:0051923"
}